positive regulation of hepatic stellate cell proliferation [GO:1904899] (biological process) Definition: Any process that activates or increases the frequency, rate or extent of hepatic stellate cell proliferation. Relationships: is a type of positive regulation of fibroblast proliferation [GO:0048146]; is a type of GO:1904897; positively regulates hepatic stellate cell proliferation [GO:1990922] References: PMID:15358192 Sources: GOC:TermGenie, GO_REF:0000058 Also known as: positive regulation of Ito cell proliferation, positive regulation of hepatic perisinusoidal cell proliferation, positive regulation of perisinusoidal cell proliferation, up regulation of Ito cell proliferation, up regulation of hepatic perisinusoidal cell proliferation, up regulation of hepatic stellate cell proliferation, up regulation of perisinusoidal cell proliferation, up-regulation of Ito cell proliferation, up-regulation of hepatic perisinusoidal cell proliferation, up-regulation of hepatic stellate cell proliferation, up-regulation of perisinusoidal cell proliferation, upregulation of Ito cell proliferation, upregulation of hepatic perisinusoidal cell proliferation, upregulation of hepatic stellate cell proliferation, upregulation of perisinusoidal cell proliferation, activation of Ito cell proliferation, activation of hepatic perisinusoidal cell proliferation, activation of hepatic stellate cell proliferation, activation of perisinusoidal cell proliferation